{
  "term_id": "GO:0005886",
  "gene_name": "Olfactory receptor 2V1",
  "gene": "UniProtKB:Q8NHB1",
  "term_label": "plasma membrane",
  "gene_symbol": "OR2V1"
}